{
  "term_id": "GO:0003700",
  "gene_symbol": "ZNF358",
  "gene": "UniProtKB:Q9NW07",
  "term_label": "DNA-binding transcription factor activity",
  "gene_name": "Zinc finger protein 358"
}